octamethylcyclotetrasiloxane catabolic process [GO:0046517] (biological process) Definition: The chemical reactions and pathways resulting in the breakdown of octamethylcyclotetrasiloxane, a cyclic silicone-oxygen ring compound with two methyl groups attached to each silicone atom. Relationships: is a type of GO:0046455 Subtypes: octamethylcyclotetrasiloxane catabolic process to dimethylsilanediol [GO:0042210] References: PMID:10224038 Sources: GOC:ai Also known as: octamethylcyclotetrasiloxane breakdown, octamethylcyclotetrasiloxane catabolism, octamethylcyclotetrasiloxane degradation